{
  "gene_name": "Calsequestrin-2",
  "gene": "UniProtKB:O14958",
  "gene_symbol": "CASQ2",
  "term_id": "GO:0010881",
  "term_label": "regulation of cardiac muscle contraction by regulation of the release of sequestered calcium ion"
}